estrogen binding [GO:0099130] (MF) Definition: Binding to an estrogen. Sources: GOC:dos Relationships: is a type of GO:0042562